regulation of neuronal synaptic plasticity [GO:0048168] (BP) Relationships: is a type of regulation of synaptic plasticity [GO:0048167] References: PMID:11891290 Sources: GOC:jid Definition: A process that modulates neuronal synaptic plasticity, the ability of neuronal synapses to change as circumstances require. They may alter function, such as increasing or decreasing their sensitivity, or they may increase or decrease in actual numbers. Note: Note that the syntax of the definition of this term is different from the usual regulation syntax because it describes regulation of a trait rather than regulation of a process. Subtypes: regulation of neuronal synaptic plasticity in response to neurotrophin [GO:0031637], regulation of long-term neuronal synaptic plasticity [GO:0048169], GO:0048172